{
  "term_label": "Unknown molecular function",
  "term_id": "UNKNOWN:0001",
  "gene_symbol": "TRAJ43",
  "gene_name": "T cell receptor alpha joining 43 (Fragment)",
  "gene": "UniProtKB:A0A075B6V1"
}